{
  "gene": "UniProtKB:Q14654",
  "gene_symbol": "KCNJ11",
  "gene_name": "ATP-sensitive inward rectifier potassium channel 11",
  "term_label": "potassium ion import across plasma membrane",
  "term_id": "GO:1990573"
}